negative regulation of synapse assembly [GO:0051964] (biological process) Sources: GOC:ai, GOC:pr Subtypes: negative regulation of synaptic assembly at neuromuscular junction [GO:0045886], negative regulation of excitatory synapse assembly [GO:1904890], negative regulation of presynapse assembly [GO:1905607], GO:1905703 Definition: Any process that stops, prevents, or reduces the frequency, rate or extent of synapse assembly, the aggregation, arrangement and bonding together of a set of components to form a synapse. Relationships: is a type of negative regulation of nervous system development [GO:0051961]; is a type of regulation of synapse assembly [GO:0051963]; is_a negative regulation of cell junction assembly [GO:1901889]; is a type of negative regulation of synapse organization [GO:1905809]; negatively regulates synapse assembly [GO:0007416] Also known as: down regulation of synapse assembly, down-regulation of synapse assembly, downregulation of synapse assembly, negative regulation of synapse biogenesis, negative regulation of synaptogenesis, inhibition of synapse assembly